{
  "gene": "UniProtKB:P49910",
  "gene_name": "Zinc finger protein 165",
  "term_id": "UNKNOWN:0003",
  "term_label": "Unknown cellular component",
  "gene_symbol": "ZNF165"
}